nonribosomal peptide biosynthetic process [GO:0019184] (biological process) Definition: The biosynthetic process in which peptide bond formation occurs in the absence of the translational machinery. Examples include the synthesis of antibiotic peptides, and glutathione. Also known as: non-ribosomal peptide biosynthesis, non-ribosomal peptide biosynthetic process, non-ribosomal peptide formation, non-ribosomal peptide synthesis, nonribosomal peptide anabolism, nonribosomal peptide biosynthesis, nonribosomal peptide formation, nonribosomal peptide synthesis, nonribosomal peptide synthetase Relationships: is a type of peptide biosynthetic process [GO:0043043] Sources: ISBN:0198506732 Subtypes: GO:0006750, siderophore biosynthetic process [GO:0019290], vancomycin biosynthetic process [GO:0033072]